{
  "gene_symbol": "RNF169",
  "gene": "UniProtKB:Q8NCN4",
  "term_label": "nucleosome binding",
  "term_id": "GO:0031491",
  "gene_name": "E3 ubiquitin-protein ligase RNF169"
}